{
  "gene_name": "ATP synthase membrane subunit K, mitochondrial",
  "term_label": "proton-transporting ATP synthase complex",
  "gene_symbol": "ATP5MK",
  "gene": "UniProtKB:Q96IX5",
  "term_id": "GO:0045259"
}